somitomeric trunk muscle development [GO:0002075] (biological process) References: PMID:16638982 Sources: GOC:dph Regulation: regulated by regulation of somitomeric trunk muscle development [GO:0014708]; positively regulated by positive regulation of somitomeric trunk muscle development [GO:0014709]; negatively regulated by negative regulation of somitomeric trunk muscle development [GO:0014710] Definition: The process whose specific outcome is the progression of the somitomeric trunk muscle over time, from its formation to the mature structure. The somitomeric trunk muscle is derived from somitomeric mesoderm. The muscle begins its development with the differentiation of the muscle cells and ends with the mature muscle. An example of this process is found in Mus musculus. Relationships: is a type of skeletal muscle organ development [GO:0060538]